{
  "term_id": "GO:0051321",
  "gene_symbol": "TUBGCP2",
  "gene": "UniProtKB:Q9BSJ2",
  "term_label": "meiotic cell cycle",
  "gene_name": "Gamma-tubulin complex component 2"
}